rRNA endonuclease activity [GO:0033902] (molecular function) Also known as: alpha-sarcin Sources: EC:4.6.1.23 Relationships: is a type of RNA endonuclease activity [GO:0004521]; is_a phosphorus-oxygen lyase activity [GO:0016849] Definition: Catalysis of the reaction: a 28S rRNA containing guanosine-adenosine pair + H2O = an [RNA fragment]-3'-adenosine-3'-phosphate + a 5'-a hydroxy-guanosine-3'-[RNA fragment].